{
  "gene_symbol": "MRM2",
  "term_label": "RNA methylation",
  "gene_name": "rRNA methyltransferase 2, mitochondrial",
  "gene": "UniProtKB:Q9UI43",
  "term_id": "GO:0001510"
}